{
  "term_label": "mitochondrial fusion",
  "gene_name": "Mitofusin-1",
  "term_id": "GO:0008053",
  "gene": "UniProtKB:Q8IWA4",
  "gene_symbol": "MFN1"
}